{
  "gene_name": "Protein Wnt-10a",
  "term_label": "extracellular space",
  "term_id": "GO:0005615",
  "gene": "UniProtKB:Q9GZT5",
  "gene_symbol": "WNT10A"
}